{
  "gene": "UniProtKB:Q6IPT2",
  "gene_symbol": "GARIN5A",
  "term_id": "UNKNOWN:0002",
  "term_label": "Unknown biological process",
  "gene_name": "Golgi-associated RAB2 interactor protein 5A"
}